{
  "gene_symbol": "TMEM106B",
  "term_id": "GO:0007040",
  "gene": "UniProtKB:Q9NUM4",
  "gene_name": "Transmembrane protein 106B",
  "term_label": "lysosome organization"
}